{
  "gene_symbol": "ZNF100",
  "term_id": "GO:0006355",
  "gene_name": "Zinc finger protein 100",
  "term_label": "regulation of DNA-templated transcription",
  "gene": "UniProtKB:Q8IYN0"
}